{
  "gene_symbol": "CDC16",
  "term_id": "GO:0051301",
  "gene_name": "Cell division cycle protein 16 homolog",
  "term_label": "cell division",
  "gene": "UniProtKB:Q13042"
}